{
  "gene_symbol": "RAB11FIP5",
  "term_label": "regulated exocytosis",
  "gene": "UniProtKB:Q9BXF6",
  "gene_name": "Rab11 family-interacting protein 5",
  "term_id": "GO:0045055"
}